SRP-dependent cotranslational protein targeting to membrane, signal sequence recognition [GO:0006617] (biological process) Relationships: is a type of protein-containing complex assembly [GO:0065003]; is part of SRP-dependent cotranslational protein targeting to membrane [GO:0006614] Sources: ISBN:0815316194 Definition: The process in which SRP binds to the signal peptide in a nascent protein, causing protein elongation to pause, during cotranslational membrane targeting. Also known as: SRP-dependent cotranslational membrane targeting, signal sequence recognition, SRP-dependent cotranslational protein-membrane targeting, signal sequence recognition, signal sequence recognition during SRP-dependent cotranslational protein targeting to membrane